{
  "gene_symbol": "NATD1",
  "term_id": "UNKNOWN:0003",
  "gene": "UniProtKB:Q8N6N6",
  "term_label": "Unknown cellular component",
  "gene_name": "Protein NATD1"
}